negative regulation of cell communication by electrical coupling [GO:0010651] (biological process) Definition: Any process that decreases the frequency, rate or extent of cell communication via electrical coupling. Cell communication via electrical coupling is the process that mediates signaling interactions between one cell and another cell by transfer of current between their adjacent cytoplasms via intercellular protein channels. Sources: GOC:dph, GOC:kmv, GOC:tb Relationships: is a type of negative regulation of cell communication [GO:0010648]; is a type of regulation of cell communication by electrical coupling [GO:0010649]; negatively regulates cell communication by electrical coupling [GO:0010644] Subtypes: negative regulation of cell communication by electrical coupling involved in cardiac conduction [GO:1901845]